nuclear lncRNA surveillance [GO:0180036] (biological process) Definition: A process that identifies and degrades defective or aberrant lncRNAs within the nucleus. Relationships: is a type of nuclear RNA surveillance [GO:0071027]; is_a GO:0110064 Sources: GOC:vw